{
  "gene_symbol": "PPP1R16A",
  "term_label": "cytoplasm",
  "term_id": "GO:0005737",
  "gene_name": "Protein phosphatase 1 regulatory subunit 16A",
  "gene": "UniProtKB:Q96I34"
}